{
  "gene_symbol": "CDNF",
  "term_label": "extracellular space",
  "gene_name": "Cerebral dopamine neurotrophic factor",
  "gene": "UniProtKB:Q49AH0",
  "term_id": "GO:0005615"
}